{
  "gene": "UniProtKB:P49756",
  "gene_symbol": "RBM25",
  "term_id": "UNKNOWN:0003",
  "term_label": "Unknown cellular component",
  "gene_name": "RNA-binding protein 25"
}